{
  "gene": "UniProtKB:Q9BW19",
  "gene_name": "Kinesin-like protein KIFC1",
  "term_id": "GO:0016887",
  "gene_symbol": "KIFC1",
  "term_label": "ATP hydrolysis activity"
}